adaxial/abaxial axis specification [GO:0009943] (biological process) Also known as: adaxial/abaxial determination Relationships: is a type of GO:0009798; is part of GO:0009955 Definition: The establishment, maintenance and elaboration of the adaxial / abaxial axis. Adaxial refers to being situated toward an axis of an anatomical structure. Abaxial refers to being situated away from an axis of an anatomical structure. Sources: GOC:dph, GOC:tb